phagosome-lysosome fusion involved in apoptotic cell clearance [GO:0090389] (biological process) Definition: The creation of a phagolysosome from a phagosome and a lysosome as a part of apoptotic cell clearance. Relationships: is a type of phagosome-lysosome fusion [GO:0090385]; is part of phagolysosome assembly involved in apoptotic cell clearance [GO:0090387] Sources: GOC:kmv, GOC:tb